perichondral ossification [GO:0036073] (biological process) Relationships: is a type of intramembranous ossification [GO:0001957] Sources: GO_REF:0000034 Definition: Intramembranous ossification from the surface of a cartilage element as the perichondrium becomes a periosteum, without replacement of cartilage.